{
  "term_id": "GO:0000932",
  "gene_symbol": "WTIP",
  "gene": "UniProtKB:A6NIX2",
  "term_label": "P-body",
  "gene_name": "Wilms tumor protein 1-interacting protein"
}